{
  "term_label": "Unknown molecular function",
  "term_id": "UNKNOWN:0001",
  "gene": "UniProtKB:A0A075B706",
  "gene_symbol": "TRDJ1",
  "gene_name": "T cell receptor delta joining 1"
}